{
  "gene": "UniProtKB:O60225",
  "gene_symbol": "SSX5",
  "term_id": "UNKNOWN:0001",
  "gene_name": "Protein SSX5",
  "term_label": "Unknown molecular function"
}